{
  "term_id": "GO:2001240",
  "gene": "UniProtKB:O95677",
  "gene_symbol": "EYA4",
  "gene_name": "Eyes absent homolog 4",
  "term_label": "negative regulation of extrinsic apoptotic signaling pathway in absence of ligand"
}